{
  "gene_symbol": "PSG11",
  "gene": "UniProtKB:Q9UQ72",
  "gene_name": "Pregnancy-specific beta-1-glycoprotein 11",
  "term_label": "homophilic cell-cell adhesion",
  "term_id": "GO:0007156"
}